cerebral cortex tangential migration using cell-cell interactions [GO:0021823] (biological process) Subtypes: postnatal olfactory bulb interneuron migration [GO:0021827] Relationships: is a type of substrate-dependent cerebral cortex tangential migration [GO:0021825] References: PMID:12626695 Sources: GOC:cls, GOC:dgh, GOC:dph, GOC:jid, GO_REF:0000021 Definition: The process in which neurons interact with each other to promote migration along a tangential plane. Also known as: chain migration